{
  "gene": "UniProtKB:Q9Y282",
  "gene_name": "Endoplasmic reticulum-Golgi intermediate compartment protein 3",
  "term_id": "GO:0005783",
  "term_label": "endoplasmic reticulum",
  "gene_symbol": "ERGIC3"
}